{
  "term_label": "RNA polymerase II transcription regulatory region sequence-specific DNA binding",
  "gene": "UniProtKB:Q6VUC0",
  "gene_name": "Transcription factor AP-2-epsilon",
  "term_id": "GO:0000977",
  "gene_symbol": "TFAP2E"
}